peptidylglycine monooxygenase activity [GO:0004504] (molecular function) Definition: Catalysis of the reaction: peptidyl-glycine + ascorbate + O2 = peptidyl(2-hydroxyglycine) + dehydroascorbate + H2O. Also known as: peptidylglycine 2-hydroxylase activity, PAM activity, PAM-A, PAM-B, peptide alpha-amidating enzyme, peptide alpha-amide synthase activity, peptide-alpha-amide synthetase activity, peptidyl alpha-amidating enzyme activity, peptidylglycine alpha-amidating monooxygenase activity, peptidylglycine alpha-hydroxylase activity, peptidylglycine,ascorbate:oxygen oxidoreductase (2-hydroxylating), synthase, peptide alpha-amide Relationships: is a type of oxidoreductase activity, acting on paired donors, with incorporation or reduction of molecular oxygen, reduced ascorbate as one donor, and incorporation of one atom of oxygen [GO:0016715] Sources: EC:1.14.17.3